{
  "gene_symbol": "ZNF131",
  "term_id": "GO:0002682",
  "term_label": "regulation of immune system process",
  "gene_name": "Zinc finger protein 131",
  "gene": "UniProtKB:P52739"
}